{
  "gene": "UniProtKB:A0A075B6N1",
  "term_id": "GO:0005886",
  "term_label": "plasma membrane",
  "gene_name": "T cell receptor beta variable 19",
  "gene_symbol": "TRBV19"
}